5-epi-aristolochene synthase activity [GO:0102698] (molecular function) Definition: Catalysis of the reaction: 2-trans,6-trans-farnesyl diphosphate = (+)-5-epi-aristolochene + diphosphoric acid. Sources: EC:4.2.3.61, GOC:pz Relationships: is a type of GO:0016838